chondro-6-sulfatase activity [GO:0033888] (MF) Sources: EC:3.1.6.10, RHEA:10536 Relationships: is_a sulfuric ester hydrolase activity [GO:0008484] Definition: Catalysis of the reaction: 4-deoxy-beta-D-gluc-4-enuronosyl-(1->3)-N-acetyl-D-galactosamine 6-sulfate + H2O = 4-deoxy-beta-D-gluc-4-enuronosyl-(1->3)-N-acetyl-D-galactosamine + H+ + sulfate. Also known as: 4-deoxy-beta-D-gluc-4-enuronosyl-(1,3)-N-acetyl-D-galactosamine-6-sulfate 6-sulfohydrolase activity